{
  "gene_symbol": "H2AJ",
  "term_id": "GO:0030527",
  "gene": "UniProtKB:Q9BTM1",
  "gene_name": "Histone H2A.J",
  "term_label": "structural constituent of chromatin"
}